{
  "gene_name": "ABI gene family member 3",
  "term_id": "GO:0030334",
  "term_label": "regulation of cell migration",
  "gene_symbol": "ABI3",
  "gene": "UniProtKB:Q9P2A4"
}